{
  "gene": "UniProtKB:Q99795",
  "term_id": "UNKNOWN:0001",
  "gene_name": "Cell surface A33 antigen",
  "term_label": "Unknown molecular function",
  "gene_symbol": "GPA33"
}